{
  "term_id": "GO:0005813",
  "gene_name": "Leucine-rich repeat-containing protein 45",
  "gene": "UniProtKB:Q96CN5",
  "term_label": "centrosome",
  "gene_symbol": "LRRC45"
}